{
  "gene_symbol": "PNPLA3",
  "term_label": "triacylglycerol lipase activity",
  "gene_name": "1-acylglycerol-3-phosphate O-acyltransferase PNPLA3",
  "gene": "UniProtKB:Q9NST1",
  "term_id": "GO:0004806"
}